{
  "term_label": "cytokine activity",
  "gene_symbol": "IFNA7",
  "gene": "UniProtKB:P01567",
  "term_id": "GO:0005125",
  "gene_name": "Interferon alpha-7"
}